{
  "gene_name": "Mastermind-like protein 1",
  "term_id": "GO:0007221",
  "term_label": "positive regulation of transcription of Notch receptor target",
  "gene_symbol": "MAML1",
  "gene": "UniProtKB:Q92585"
}